{
  "gene": "UniProtKB:Q12918",
  "gene_name": "Killer cell lectin-like receptor subfamily B member 1",
  "gene_symbol": "KLRB1",
  "term_label": "regulation of natural killer cell mediated cytotoxicity",
  "term_id": "GO:0042269"
}